{
  "gene_name": "Vitrin",
  "gene": "UniProtKB:Q6UXI7",
  "term_label": "Unknown molecular function",
  "term_id": "UNKNOWN:0001",
  "gene_symbol": "VIT"
}